protein trimerization [GO:0070206] (biological process) Subtypes: protein homotrimerization [GO:0070207], protein heterotrimerization [GO:0070208] Definition: The formation of a protein trimer, a macromolecular structure consisting of three noncovalently associated identical or nonidentical subunits. Sources: GOC:hjd Relationships: is_a protein complex oligomerization [GO:0051259] Also known as: protein trimer assembly, protein trimer biosynthesis, protein trimer biosynthetic process, protein trimer formation